{
  "term_label": "sensory perception of pain",
  "gene": "UniProtKB:P41145",
  "term_id": "GO:0019233",
  "gene_name": "Kappa-type opioid receptor",
  "gene_symbol": "OPRK1"
}